{
  "gene": "UniProtKB:Q9NRP0",
  "term_id": "GO:0030674",
  "term_label": "protein-macromolecule adaptor activity",
  "gene_name": "Oligosaccharyltransferase complex subunit OSTC",
  "gene_symbol": "OSTC"
}